{
  "gene_name": "Adenosine 3'-phospho 5'-phosphosulfate transporter 1",
  "term_id": "GO:0046964",
  "term_label": "3'-phosphoadenosine 5'-phosphosulfate transmembrane transporter activity",
  "gene": "UniProtKB:Q8TB61",
  "gene_symbol": "SLC35B2"
}